extracellular matrix protein binding [GO:1990430] (MF) Relationships: is a type of protein binding [GO:0005515] Definition: Binding to a protein that is part of an extracellular matrix. References: PMID:22355679